negative regulation of Ras protein signal transduction [GO:0046580] (biological process) Definition: Any process that stops, prevents, or reduces the frequency, rate or extent of Ras protein signal transduction. Also known as: down regulation of Ras protein signal transduction, down-regulation of Ras protein signal transduction, downregulation of Ras protein signal transduction, inhibition of Ras protein signal transduction Relationships: is a type of regulation of Ras protein signal transduction [GO:0046578]; is a type of negative regulation of small GTPase mediated signal transduction [GO:0051058]; negatively regulates Ras protein signal transduction [GO:0007265] Sources: GOC:bf